genital disc development [GO:0035215] (biological process) Definition: Progression of the genital imaginal disc over time, from its initial formation through to its metamorphosis to form the adult terminalia, comprising the entire set of internal and external genitalia and analia. Both sexes of Drosophila have a single genital disc formed from the female and male genital primordia, and the anal primordium. The anal primordium develops in both sexes, forming either male or female analia. However, only one of the genital primordia develops in each sex, forming either the male or the female genitalia. Relationships: is a type of imaginal disc development [GO:0007444] References: PMID:11494318 Sources: GOC:bf, ISBN:0879694238